{
  "term_id": "GO:0000977",
  "gene_symbol": "DUX4L2",
  "term_label": "RNA polymerase II transcription regulatory region sequence-specific DNA binding",
  "gene": "UniProtKB:P0CJ85",
  "gene_name": "Double homeobox protein 4-like protein 2"
}